{
  "gene_name": "Zinc finger protein 335",
  "gene_symbol": "ZNF335",
  "term_label": "brain development",
  "gene": "UniProtKB:Q9H4Z2",
  "term_id": "GO:0007420"
}